vacuolar transmembrane transport [GO:0034486] (biological process) Subtypes: amino acid transmembrane export from vacuole [GO:0032974], amino acid transmembrane import into vacuole [GO:0032975], cadmium ion import into vacuole [GO:0036249], GO:0071995, glutathione transmembrane import into vacuole [GO:0071996], L-aspartate transmembrane export from vacuole [GO:0089703], molybdate ion export from vacuole [GO:0090414], aspartate transmembrane import into vacuole [GO:0090453], GO:0090455, GO:0140145, GO:0140146, GO:0140147, heme export from vacuole to cytoplasm [GO:0140357], zinc ion import into lysosome [GO:0140916], purine nucleotide import into lysosome [GO:0141013], transmembrane transport from lysosomal lumen to cytosol [GO:0170063], polyphosphate import into vacuole [GO:0180042], fructose export from vacuole to cytoplasm [GO:1902334], GO:1905011 Relationships: is a type of transmembrane transport [GO:0055085] Sources: GOC:mah Note: Note that this term is not intended for use in annotating lateral movement within membranes. Also known as: vacuolar membrane transport Definition: The process in which a solute is transported from one side of the vacuolar membrane to the other.